{
  "term_id": "GO:0062081",
  "gene_symbol": "KLRC4",
  "gene": "UniProtKB:O43908",
  "term_label": "activating MHC class Ib receptor activity",
  "gene_name": "NKG2-F type II integral membrane protein"
}